{
  "gene": "UniProtKB:Q9H094",
  "term_id": "UNKNOWN:0001",
  "gene_symbol": "NBPF3",
  "gene_name": "Neuroblastoma breakpoint family member 3",
  "term_label": "Unknown molecular function"
}